negative regulation of tridecane biosynthetic process [GO:1900885] (biological process) Sources: GOC:TermGenie, GOC:mengo_curators Definition: Any process that stops, prevents or reduces the frequency, rate or extent of tridecane biosynthetic process. Also known as: down regulation of tridecane anabolism, down regulation of tridecane biosynthesis, down regulation of tridecane biosynthetic process, down regulation of tridecane formation, down regulation of tridecane synthesis, down-regulation of tridecane anabolism, down-regulation of tridecane biosynthesis, down-regulation of tridecane biosynthetic process, down-regulation of tridecane formation, down-regulation of tridecane synthesis, downregulation of tridecane anabolism, downregulation of tridecane biosynthesis, downregulation of tridecane biosynthetic process, downregulation of tridecane formation, downregulation of tridecane synthesis, negative regulation of tridecane anabolism, negative regulation of tridecane biosynthesis, negative regulation of tridecane formation, negative regulation of tridecane synthesis, inhibition of tridecane anabolism, inhibition of tridecane biosynthesis, inhibition of tridecane biosynthetic process, inhibition of tridecane formation, inhibition of tridecane synthesis Relationships: is a type of regulation of tridecane biosynthetic process [GO:1900884]; is a type of GO:1901578; negatively regulates GO:1900632